{
  "gene": "UniProtKB:Q13634",
  "term_id": "GO:0000902",
  "gene_symbol": "CDH18",
  "gene_name": "Cadherin-18",
  "term_label": "cell morphogenesis"
}